{
  "gene_symbol": "MTSS2",
  "gene_name": "Protein MTSS 2",
  "term_id": "GO:0061024",
  "term_label": "membrane organization",
  "gene": "UniProtKB:Q765P7"
}